positive regulation of nucleotide-binding oligomerization domain containing 1 signaling pathway [GO:0070430] (biological process) Also known as: positive regulation of NOD1 signaling pathway, positive regulation of nucleotide-binding oligomerization domain containing 1 signalling pathway Relationships: is a type of positive regulation of nucleotide-binding domain, leucine rich repeat containing receptor signaling pathway [GO:0070426]; is a type of regulation of nucleotide-binding oligomerization domain containing 1 signaling pathway [GO:0070428]; positively regulates nucleotide-binding oligomerization domain containing 1 signaling pathway [GO:0070427] Sources: GOC:add Definition: Any process that activates or increases the frequency, rate, or extent of the nucleotide-binding oligomerization domain containing 1 (NOD1) pathway.